{
  "term_id": "GO:0004674",
  "term_label": "protein serine/threonine kinase activity",
  "gene": "UniProtKB:Q13153",
  "gene_name": "Serine_threonine-protein kinase PAK 1",
  "gene_symbol": "PAK1"
}